negative regulation of cAMP-dependent protein kinase activity [GO:2000480] (biological process) Definition: Any process that stops, prevents or reduces the frequency, rate or extent of cAMP-dependent protein kinase activity. Relationships: is a type of negative regulation of protein serine/threonine kinase activity [GO:0071901]; is a type of GO:2000479; negatively regulates cAMP-dependent protein kinase activity [GO:0004691] Also known as: negative regulation of 3',5' cAMP-dependent protein kinase activity, negative regulation of 3',5'-cAMP-dependent protein kinase activity, negative regulation of ATP:protein phosphotransferase (cAMP-dependent) activity, negative regulation of adenosine 3',5'-cyclophosphate-dependent protein kinase activity, negative regulation of cAMP-dependent protein kinase, intrinsic catalyst activity, negative regulation of cyclic AMP-dependent protein kinase activity, negative regulation of AMPK, negative regulation of PKA, negative regulation of PKA C, negative regulation of STK22, negative regulation of protein kinase A activity Sources: GOC:obol